{
  "term_label": "leukocyte migration involved in inflammatory response",
  "gene_symbol": "ELANE",
  "term_id": "GO:0002523",
  "gene_name": "Neutrophil elastase",
  "gene": "UniProtKB:P08246"
}